{
  "term_label": "glycerol channel activity",
  "gene_name": "Aquaporin-3",
  "term_id": "GO:0015254",
  "gene": "UniProtKB:Q92482",
  "gene_symbol": "AQP3"
}